{
  "gene": "UniProtKB:Q8IV20",
  "gene_name": "Purine nucleoside phosphorylase LACC1",
  "term_id": "UNKNOWN:0003",
  "gene_symbol": "LACC1",
  "term_label": "Unknown cellular component"
}